maturation of LSU-rRNA from tetracistronic rRNA transcript (SSU-rRNA, 5.8S rRNA, 2S rRNA, LSU-rRNA) [GO:0000473] (biological process) Relationships: is_a maturation of LSU-rRNA [GO:0000470] Sources: GOC:curators Definition: Any process involved in the maturation of a precursor Large SubUnit (LSU) ribosomal RNA (rRNA) molecule into a mature LSU-rRNA molecule from the pre-rRNA molecule originally produced as a tetracistronic rRNA transcript that contains the Small Subunit (SSU) rRNA, 5.8 S rRNA, 2S rRNA, and Large Subunit (LSU) in that order from 5' to 3' along the primary transcript.